{
  "term_id": "UNKNOWN:0001",
  "gene_symbol": "MUC22",
  "term_label": "Unknown molecular function",
  "gene": "UniProtKB:E2RYF6",
  "gene_name": "Mucin-22"
}